{
  "gene": "UniProtKB:O43502",
  "gene_name": "DNA repair protein RAD51 homolog 3",
  "gene_symbol": "RAD51C",
  "term_id": "GO:0000707",
  "term_label": "meiotic DNA recombinase assembly"
}